DNA photolyase activity [GO:0003913] (molecular function) Subtypes: deoxyribodipyrimidine photo-lyase activity [GO:0003904], DNA (6-4) photolyase activity [GO:0003914] Relationships: is a type of GO:0016830; is a type of GO:0140097 Definition: Catalysis of the repair of a photoproduct resulting from ultraviolet irradiation of two adjacent pyrimidine residues in DNA. References: PMID:11124949 Sources: GOC:mah